glycine formimidoyltransferase activity [GO:0030408] (molecular function) Also known as: formimidoyltransferase activity, formiminotransferase activity, glycine formiminotransferase activity, 5-formimidoyltetrahydrofolate:glycine N-formimidoyltransferase activity, FIG formiminotransferase activity, formiminoglycine formiminotransferase activity Relationships: is a type of hydroxymethyl-, formyl- and related transferase activity [GO:0016742] Definition: Catalysis of the reaction: 5-formimidoyltetrahydrofolate + glycine = (6S)-5,6,7,8-tetrahydrofolate + N-formimidoylglycine. Sources: RHEA:24288